{
  "gene_symbol": "DCT",
  "gene_name": "L-dopachrome tautomerase",
  "gene": "UniProtKB:P40126",
  "term_label": "dopachrome isomerase activity",
  "term_id": "GO:0004167"
}